{
  "gene_symbol": "ADAM20",
  "gene_name": "Disintegrin and metalloproteinase domain-containing protein 20",
  "gene": "UniProtKB:O43506",
  "term_id": "GO:1990913",
  "term_label": "sperm head plasma membrane"
}